dolichol-phosphate-mannose synthase regulator activity [GO:0097713] (molecular function) Definition: Binds to and modulates the activity of dolichol-phosphate-mannose synthase. References: PMID:10835346 Sources: GOC:vw Relationships: is_a enzyme regulator activity [GO:0030234]; regulates GO:0004169